{
  "gene_symbol": "LINC00869",
  "term_id": "UNKNOWN:0002",
  "gene_name": "Putative uncharacterized protein encoded by LINC00869",
  "term_label": "Unknown biological process",
  "gene": "UniProtKB:P0C866"
}